{
  "gene_symbol": "REXO2",
  "term_id": "GO:0000175",
  "gene_name": "Oligoribonuclease, mitochondrial",
  "gene": "UniProtKB:Q9Y3B8",
  "term_label": "3'-5'-RNA exonuclease activity"
}